{
  "term_id": "UNKNOWN:0002",
  "gene_symbol": "CCDC140",
  "term_label": "Unknown biological process",
  "gene": "UniProtKB:Q96MF4",
  "gene_name": "Coiled-coil domain-containing protein 140"
}